{
  "term_label": "phosphate transmembrane transporter activity",
  "gene_symbol": "SLC20A1",
  "gene": "UniProtKB:Q8WUM9",
  "term_id": "GO:0005315",
  "gene_name": "Sodium-dependent phosphate transporter 1"
}